{
  "term_id": "GO:0031032",
  "gene_symbol": "ROCK1",
  "gene_name": "Rho-associated protein kinase 1",
  "term_label": "actomyosin structure organization",
  "gene": "UniProtKB:Q13464"
}